{
  "gene_name": "Pro-cathepsin H",
  "term_id": "GO:0006955",
  "gene": "UniProtKB:P09668",
  "term_label": "immune response",
  "gene_symbol": "CTSH"
}